{
  "gene_symbol": "CWC25",
  "term_id": "GO:0000398",
  "gene_name": "Pre-mRNA-splicing factor CWC25 homolog",
  "term_label": "mRNA splicing, via spliceosome",
  "gene": "UniProtKB:Q9NXE8"
}